{
  "term_label": "terminal bouton",
  "term_id": "GO:0043195",
  "gene_symbol": "SLC18A2",
  "gene_name": "Synaptic vesicular amine transporter",
  "gene": "UniProtKB:Q05940"
}